uterine gland development [GO:1903709] (biological process) Also known as: endometrial gland development, endometrium gland development, uterine glands development, uterine glands set development, glandulae uterinae development, glandular part of endometrium development, set of uterine glands development References: PMID:23619340 Sources: GOC:TermGenie, GO_REF:0000094 Definition: The process whose specific outcome is the progression of an uterine gland over time, from its formation to the mature structure. Relationships: is a type of GO:0048732